{
  "term_label": "structural constituent of eye lens",
  "gene_name": "Beta-crystallin B3",
  "gene": "UniProtKB:P26998",
  "gene_symbol": "CRYBB3",
  "term_id": "GO:0005212"
}